{
  "term_id": "GO:0001972",
  "term_label": "retinoic acid binding",
  "gene_name": "Cellular retinoic acid-binding protein 2",
  "gene_symbol": "CRABP2",
  "gene": "UniProtKB:P29373"
}